lateral cell cortex [GO:0097575] (cellular component) Definition: The region directly beneath the plasma membrane of the lateral portion of the cell. References: PMID:24146635 Sources: GOC:mah Relationships: is a type of cell cortex region [GO:0099738]; is part of lateral part of cell [GO:0097574]